detection of muscle activity involved in regulation of muscle adaptation [GO:0014875] (BP) Definition: The series of events by which a muscle activity stimulus is received and converted into a molecular signal. This occurs as part of the regulation of muscle adaptation. Sources: GOC:ef, GOC:mtg_muscle Also known as: detection of fatigue Relationships: is a type of GO:0014864; is a type of GO:0014873